{
  "term_id": "GO:0005886",
  "gene_symbol": "TTC7B",
  "gene": "UniProtKB:Q86TV6",
  "term_label": "plasma membrane",
  "gene_name": "Tetratricopeptide repeat protein 7B"
}